{
  "gene": "UniProtKB:P51674",
  "term_id": "GO:0031175",
  "gene_name": "Neuronal membrane glycoprotein M6-a",
  "term_label": "neuron projection development",
  "gene_symbol": "GPM6A"
}